{
  "gene_symbol": "RNF14",
  "term_id": "GO:0031624",
  "gene_name": "E3 ubiquitin-protein ligase RNF14",
  "term_label": "ubiquitin conjugating enzyme binding",
  "gene": "UniProtKB:Q9UBS8"
}